erythrocyte apoptotic process [GO:1902217] (biological process) Regulation: regulated by regulation of erythrocyte apoptotic process [GO:1902250]; negatively regulated by negative regulation of erythrocyte apoptotic process [GO:1902251]; positively regulated by positive regulation of erythrocyte apoptotic process [GO:1902252] Relationships: is_a myeloid cell apoptotic process [GO:0033028] Also known as: RBC apoptotic process, red blood cell apoptotic process, RBC apoptosis, erythrocyte apoptosis, red blood cell apoptosis Definition: Any apoptotic process in an erythrocyte. References: PMID:14569084 Sources: GOC:BHF, GOC:TermGenie, GOC:mtg_apoptosis, GOC:rl